{
  "gene_name": "T cell receptor alpha variable 5",
  "term_id": "UNKNOWN:0003",
  "gene": "UniProtKB:A0A0B4J249",
  "term_label": "Unknown cellular component",
  "gene_symbol": "TRAV5"
}